salicin transmembrane transporter activity [GO:0042950] (molecular function) Relationships: is a type of beta-glucoside transmembrane transporter activity [GO:0015573]; is a type of alcohol transmembrane transporter activity [GO:0015665]; is part of salicin transport [GO:0042948] Definition: Enables the transfer of salicin (saligenin-beta-D-glucopyranoside), a glucoside of o-hydroxybenzylalcohol, from one side of a membrane to the other. Sources: GOC:jl, GOC:mtg_transport, ISBN:0815340729